{
  "gene": "UniProtKB:Q9NZ20",
  "term_label": "Unknown molecular function",
  "gene_symbol": "PLA2G3",
  "gene_name": "Group 3 secretory phospholipase A2",
  "term_id": "UNKNOWN:0001"
}